platelet dense granule lumen [GO:0031089] (cellular component) Definition: The volume enclosed by the membrane of the platelet dense granule. Relationships: is a type of GO:0034774; is part of platelet dense granule [GO:0042827] Sources: GOC:mah